outer mitochondrial membrane organization [GO:0007008] (biological process) Subtypes: GO:0045040, mitochondrial outer membrane fusion [GO:1990626] Note: See also the cellular component term 'mitochondrial outer membrane ; GO:0005741'. Also known as: outer mitochondrial membrane organisation, outer mitochondrial membrane organization and biogenesis Relationships: is a type of mitochondrial membrane organization [GO:0007006] Sources: GOC:ai, GOC:dph, GOC:jl, GOC:mah Definition: A process that is carried out at the cellular level which results in the assembly, arrangement of constituent parts, or disassembly of the mitochondrial outer membrane.